{
  "gene_name": "AP-4 complex subunit mu-1",
  "gene": "UniProtKB:O00189",
  "gene_symbol": "AP4M1",
  "term_label": "clathrin adaptor activity",
  "term_id": "GO:0035615"
}